mRNA metabolic process [GO:0016071] (biological process) Also known as: mRNA metabolism Definition: The chemical reactions and pathways involving mRNA, messenger RNA, which is responsible for carrying the coded genetic 'message', transcribed from DNA, to sites of protein assembly at the ribosomes. Regulation: regulated by regulation of mRNA metabolic process [GO:1903311]; negatively regulated by negative regulation of mRNA metabolic process [GO:1903312]; positively regulated by positive regulation of mRNA metabolic process [GO:1903313] Relationships: is_a GO:0016070 Subtypes: mRNA processing [GO:0006397], mRNA catabolic process [GO:0006402], histone mRNA metabolic process [GO:0008334], GO:0009299, mRNA modification [GO:0016556], mRNA methylguanosine-cap decapping [GO:0110156], cytosolic mRNA polyadenylation [GO:0180011] Sources: ISBN:0198506732